{
  "term_label": "alanine-tRNA ligase activity",
  "term_id": "GO:0004813",
  "gene_symbol": "AARS1",
  "gene": "UniProtKB:P49588",
  "gene_name": "Alanine--tRNA ligase, cytoplasmic"
}